{
  "term_id": "UNKNOWN:0001",
  "term_label": "Unknown molecular function",
  "gene_symbol": "SERINC5",
  "gene_name": "Serine incorporator 5",
  "gene": "UniProtKB:Q86VE9"
}